regulation of interleukin-4-dependent isotype switching to IgE isotypes [GO:2000571] (biological process) Relationships: is a type of GO:0048293; RO_0002211 interleukin-4-dependent isotype switching to IgE isotypes [GO:0035708] Definition: Any process that modulates the frequency, rate or extent of interleukin-4-dependent isotype switching to IgE isotypes. Sources: GOC:obol Subtypes: GO:2000572 Also known as: regulation of IL-4-dependent isotype switching to IgE isotypes